regulation of activin receptor signaling pathway [GO:0032925] (biological process) Relationships: is a type of regulation of transmembrane receptor protein serine/threonine kinase signaling pathway [GO:0090092]; regulates activin receptor signaling pathway [GO:0032924] Definition: Any process that modulates the frequency, rate or extent of the activity of any activin receptor signaling pathway. Also known as: regulation of activin receptor signalling pathway, regulation of activin signaling pathway, regulation of activin signalling pathway Subtypes: negative regulation of activin receptor signaling pathway [GO:0032926], positive regulation of activin receptor signaling pathway [GO:0032927], regulation of nodal signaling pathway [GO:1900107] Sources: GOC:BHF, GOC:rl